monoatomic ion transport [GO:0006811] (biological process) Subtypes: monoatomic cation transport [GO:0006812], monoatomic anion transport [GO:0006820], monoatomic ion transmembrane transport [GO:0034220] Relationships: is a type of GO:0006810 Sources: GOC:ai Also known as: ion transport Regulation: regulated by regulation of monoatomic ion transport [GO:0043269]; positively regulated by positive regulation of monoatomic ion transport [GO:0043270]; negatively regulated by negative regulation of monoatomic ion transport [GO:0043271] Definition: The directed movement of a monoatomic ion into, out of or within a cell, or between cells, by means of some agent such as a transporter or pore. Monatomic ions (also called simple ions) are ions consisting of exactly one atom.